BLOC complex [GO:0031082] (cellular component) Subtypes: BLOC-1 complex [GO:0031083], BLOC-2 complex [GO:0031084], BLOC-3 complex [GO:0031085] Definition: Any of several protein complexes required for the biogenesis of specialized organelles of the endosomal-lysosomal system, such as melanosomes, platelet dense granules, and other related organelles; acronym for biogenesis of lysosomal-related organelles complex. References: PMID:15102850, PMID:15261680 Relationships: is_a GO:0140535 Also known as: BLOC-1 related complex